low-density lipoprotein particle binding [GO:0030169] (molecular function) Definition: Binding to a low-density lipoprotein particle, a lipoprotein particle that is rich in cholesterol esters and low in triglycerides, is typically composed of APOB100 and APOE, and has a density of 1.02-1.06 g/ml and a diameter of between 20-25 nm. Sources: GOC:mah Also known as: LDL binding Relationships: is a type of lipoprotein particle binding [GO:0071813]